{
  "gene": "UniProtKB:Q9P298",
  "gene_name": "HIG1 domain family member 1B",
  "term_id": "UNKNOWN:0001",
  "gene_symbol": "HIGD1B",
  "term_label": "Unknown molecular function"
}